{
  "gene_name": "EH domain-containing protein 1",
  "gene_symbol": "EHD1",
  "term_id": "GO:0006897",
  "gene": "UniProtKB:Q9H4M9",
  "term_label": "endocytosis"
}